{
  "gene": "UniProtKB:P59047",
  "term_id": "GO:0050727",
  "term_label": "regulation of inflammatory response",
  "gene_name": "NACHT, LRR and PYD domains-containing protein 5",
  "gene_symbol": "NLRP5"
}